{
  "gene": "UniProtKB:Q12866",
  "gene_symbol": "MERTK",
  "term_label": "cell surface receptor protein tyrosine kinase signaling pathway",
  "gene_name": "Tyrosine-protein kinase Mer",
  "term_id": "GO:0007169"
}